release of matrix enzymes from mitochondria [GO:0032976] (biological process) Relationships: is a type of apoptotic mitochondrial changes [GO:0008637] Note: Annotation to this term should be done with caution, particularly if the mechanism is not well clarified. References: PMID:9843949 Sources: GOC:mah, GOC:mtg_apoptosis Definition: The process in which enzymes, such as aspartate aminotransferase, are enabled to move from the mitochondrial matrix into the cytosol, as part of the apoptotic process. Also known as: mAST release from mitochondria, release of aspartate aminotransferase from mitochondria